{
  "gene_name": "Protein NEDD1",
  "gene": "UniProtKB:Q8NHV4",
  "gene_symbol": "NEDD1",
  "term_id": "GO:0007020",
  "term_label": "microtubule nucleation"
}